{
  "term_label": "olfactory receptor activity",
  "gene_symbol": "OR7A2P",
  "gene_name": "Putative olfactory receptor 7A2",
  "term_id": "GO:0004984",
  "gene": "UniProtKB:Q8NGA2"
}